6-acetylglucose deacetylase activity [GO:0047593] (molecular function) Sources: EC:3.1.1.33, RHEA:18485 Also known as: 6-O-acetylglucose deacetylase activity, 6-acetyl-D-glucose acetylhydrolase activity Relationships: is a type of deacetylase activity [GO:0019213]; is a type of carboxylic ester hydrolase activity [GO:0052689] Definition: Catalysis of the reaction: 6-acetyl-D-glucose + H2O = D-glucose + acetate + H+.